{
  "gene_name": "Protein EURL homolog",
  "gene_symbol": "EURL",
  "term_label": "Unknown cellular component",
  "term_id": "UNKNOWN:0003",
  "gene": "UniProtKB:Q9NYK6"
}